{
  "term_label": "nucleus",
  "gene_name": "Pre-B-cell leukemia transcription factor 4",
  "term_id": "GO:0005634",
  "gene_symbol": "PBX4",
  "gene": "UniProtKB:Q9BYU1"
}